sodium ion export across plasma membrane [GO:0036376] (biological process) Relationships: is a type of GO:0035725; is a type of GO:0140115 Regulation: regulated by regulation of sodium ion export across plasma membrane [GO:1903276]; negatively regulated by negative regulation of sodium ion export across plasma membrane [GO:1903277]; positively regulated by GO:1903278 Also known as: sodium ion export from cell, sodium export, sodium ion export Definition: The directed movement of sodium ions from inside of a cell, across the plasma membrane and into the extracellular region. References: PMID:14674689 Sources: GOC:vw